cellular response to puromycin [GO:1905795] (BP) References: PMID:25736288 Sources: GOC:TermGenie, GO_REF:0000071 Relationships: is a type of cellular response to nitrogen compound [GO:1901699]; is a type of GO:1901701; is a type of response to puromycin [GO:1905794] Definition: Any process that results in a change in state or activity of a cell (in terms of movement, secretion, enzyme production, gene expression, etc.) as a result of a puromycin stimulus. Also known as: cellular response to 3'-deoxy-N,N-dimethyl-3'-(O-methyl-L-tyrosinamido)adenosine